circadian regulation of systemic arterial blood pressure by the suprachiasmatic nucleus [GO:0003054] (biological process) Also known as: SCN regulation of blood pressure, master pacemaker clock regulation of blood pressure Relationships: is a type of nervous system process involved in regulation of systemic arterial blood pressure [GO:0001976]; is a type of circadian regulation of systemic arterial blood pressure [GO:0003052] Sources: GOC:mtg_cardio, GOC:rl Definition: The process in which the suprachiasmatic nucleus modulates blood pressure at different values with a regularity of approximately 24 hours.